{
  "term_label": "Unknown cellular component",
  "gene_name": "Beta-chimaerin",
  "gene": "UniProtKB:P52757",
  "term_id": "UNKNOWN:0003",
  "gene_symbol": "CHN2"
}